{
  "term_label": "cilium assembly",
  "gene_symbol": "ABLIM3",
  "gene_name": "Actin-binding LIM protein 3",
  "gene": "UniProtKB:O94929",
  "term_id": "GO:0060271"
}